{
  "term_label": "cortical actin cytoskeleton",
  "gene_name": "Protein Shroom3",
  "gene_symbol": "SHROOM3",
  "gene": "UniProtKB:Q8TF72",
  "term_id": "GO:0030864"
}